{
  "gene_symbol": "NINJ2",
  "gene": "UniProtKB:Q9NZG7",
  "term_label": "plasma membrane",
  "term_id": "GO:0005886",
  "gene_name": "Ninjurin-2"
}